receptor serine/threonine kinase binding [GO:0033612] (molecular function) Definition: Binding to a receptor that possesses protein serine/threonine kinase activity. Sources: GOC:mah Also known as: transmembrane receptor protein serine/threonine kinase ligand binding Relationships: is a type of signaling receptor binding [GO:0005102] Subtypes: transmembrane receptor protein serine/threonine kinase binding [GO:0070696]